{
  "gene_name": "Peroxisomal membrane protein 11A",
  "term_id": "GO:0005778",
  "gene_symbol": "PEX11A",
  "term_label": "peroxisomal membrane",
  "gene": "UniProtKB:O75192"
}